{
  "term_label": "RNA polymerase II cis-regulatory region sequence-specific DNA binding",
  "gene": "UniProtKB:Q0VGE8",
  "gene_symbol": "ZNF816",
  "term_id": "GO:0000978",
  "gene_name": "Zinc finger protein 816"
}